{
  "gene": "UniProtKB:Q8TD07",
  "gene_name": "Retinoic acid early transcript 1E",
  "term_label": "antigen processing and presentation of endogenous peptide antigen via MHC class Ib",
  "gene_symbol": "RAET1E",
  "term_id": "GO:0002476"
}